heterocyst development [GO:0043158] (biological process) References: PMID:11121783, PMID:35744626 Also known as: heterocyst formation, heterocyst cell differentiation, heterocyst differentiation Definition: The cellular developmental process by which a cell becomes a heterocyst, a cell that carries out nitrogen fixation. This process involves changes to the cell wall, expression of nitrogenase and other proteins involved in nitrogen fixation, and degradation of photosystem II, which produces oxygen. This process is known to occur in some cyanobacteria. Relationships: is a type of cellular developmental process [GO:0048869]